histone H3K56 deacetylase activity, NAD-dependent [GO:0140765] (molecular function) Also known as: NAD-dependent histone H3-K56 deacetylase activity, NAD-dependent histone H3K56 deacetylase activity, NAD-dependent histone deacetylase activity (H3-K56 specific) Relationships: is a type of histone deacetylase activity, NAD-dependent [GO:0017136]; is a type of histone H3K deacetylase activity [GO:0141050] Note: Comment: Note that the residue position corresponds to the canonical human H3 histone (UniProtKB:P84243); this residue is conserved across all eukaryotes. Residue 1 is the first residue following removal of the initiating Methionine (Met). Note that each histone is encoded by multiple genes, and sequences may vary across different genes within an organism. Definition: Catalysis of the reaction: histone H3 N6-acetyl-L-lysine (position 56) + NAD+ + H2O = histone H3 L-lysine (position 56) + 2''-O-acetyl-ADP-D-ribose + nicotinamide. This reaction transfers an acetyl group attached to a lysine residue in H3K56 to NAD, producing nicotinamide. References: PMID:23911928, PMID:30374165